ligase activity, forming carbon-carbon bonds [GO:0016885] (molecular function) Sources: EC:6.4.-.- Subtypes: GO:0004736, CoA carboxylase activity [GO:0016421], acetone carboxylase activity [GO:0018710], 2-oxoglutarate carboxylase activity [GO:0034029] Definition: Catalysis of the joining of two molecules via a carbon-carbon bond, with the concomitant hydrolysis of the diphosphate bond in ATP or a similar triphosphate. Relationships: is a type of GO:0016874